{
  "term_id": "GO:0019886",
  "term_label": "antigen processing and presentation of exogenous peptide antigen via MHC class II",
  "gene_name": "HLA class II histocompatibility antigen, DO beta chain",
  "gene_symbol": "HLA-DOB",
  "gene": "UniProtKB:P13765"
}